{
  "term_label": "Unknown cellular component",
  "term_id": "UNKNOWN:0003",
  "gene_name": "Alpha-1,3-mannosyl-glycoprotein 4-beta-N-acetylglucosaminyltransferase C",
  "gene": "UniProtKB:Q9UBM8",
  "gene_symbol": "MGAT4C"
}